{
  "gene_symbol": "CHRNB1",
  "term_id": "GO:0095500",
  "gene": "UniProtKB:P11230",
  "term_label": "acetylcholine receptor signaling pathway",
  "gene_name": "Acetylcholine receptor subunit beta"
}